{
  "gene": "UniProtKB:O95263",
  "term_label": "positive regulation of ERK1 and ERK2 cascade",
  "term_id": "GO:0070374",
  "gene_symbol": "PDE8B",
  "gene_name": "High affinity cAMP-specific and IBMX-insensitive 3',5'-cyclic phosphodiesterase 8B"
}